negative regulation of lamellipodium organization [GO:1902744] (biological process) Relationships: is a type of GO:0031345; is a type of regulation of lamellipodium organization [GO:1902743]; negatively regulates lamellipodium organization [GO:0097581] Subtypes: GO:0010593, GO:2000393 Also known as: down regulation of lamellipodium organization, down-regulation of lamellipodium organization, downregulation of lamellipodium organization, inhibition of lamellipodium organization Definition: Any process that stops, prevents or reduces the frequency, rate or extent of lamellipodium organization. References: PMID:16054028 Sources: GOC:TermGenie, GOC:als, GO_REF:0000058